{
  "gene_symbol": "CHD8",
  "term_label": "chromatin binding",
  "gene": "UniProtKB:Q9HCK8",
  "term_id": "GO:0003682",
  "gene_name": "Chromodomain-helicase-DNA-binding protein 8"
}